{
  "term_label": "protein catabolic process",
  "gene_symbol": "UCHL1",
  "gene_name": "Ubiquitin carboxyl-terminal hydrolase isozyme L1",
  "gene": "UniProtKB:P09936",
  "term_id": "GO:0030163"
}